{
  "gene_symbol": "CLEC16A",
  "gene_name": "Protein CLEC16A",
  "term_id": "UNKNOWN:0001",
  "term_label": "Unknown molecular function",
  "gene": "UniProtKB:Q2KHT3"
}